{
  "gene": "UniProtKB:Q13231",
  "gene_symbol": "CHIT1",
  "term_id": "GO:0004568",
  "term_label": "chitinase activity",
  "gene_name": "Chitotriosidase-1"
}